{
  "term_label": "plasma membrane",
  "gene_symbol": "GYPB",
  "gene": "UniProtKB:P06028",
  "gene_name": "Glycophorin-B",
  "term_id": "GO:0005886"
}